{
  "term_id": "GO:0031252",
  "gene_symbol": "SHTN1",
  "gene": "UniProtKB:A0MZ66",
  "term_label": "cell leading edge",
  "gene_name": "Shootin-1"
}